{
  "term_label": "calcium ion binding",
  "gene_name": "Calcium uptake protein 1, mitochondrial",
  "term_id": "GO:0005509",
  "gene": "UniProtKB:Q9BPX6",
  "gene_symbol": "MICU1"
}